{
  "gene_symbol": "EIF4E3",
  "gene": "UniProtKB:Q8N5X7",
  "term_label": "translational initiation",
  "gene_name": "Eukaryotic translation initiation factor 4E type 3",
  "term_id": "GO:0006413"
}